isoflavonoid metabolic process [GO:0046287] (biological process) Subtypes: isoflavonoid biosynthetic process [GO:0009717], GO:0046288 Definition: The chemical reactions and pathways involving isoflavonoids, a group of water-soluble phenolic derivatives, isomeric with flavonoids, containing a flavan skeleton. They are differentiated from flavonoids by the point of attachment of the aromatic ring group. Relationships: is a type of phenylpropanoid metabolic process [GO:0009698] References: PMID:15734910 Sources: GOC:ai Also known as: isoflavonoid metabolism